{
  "term_label": "Unknown cellular component",
  "gene_symbol": "TMEM212",
  "gene": "UniProtKB:A6NML5",
  "gene_name": "Transmembrane protein 212",
  "term_id": "UNKNOWN:0003"
}